positive regulation of sarcomere organization [GO:0060298] (biological process) Sources: GOC:BHF, GOC:dph, GOC:tb Also known as: positive regulation of sarcomere organisation Relationships: is a type of GO:0051155; is a type of positive regulation of cytoskeleton organization [GO:0051495]; is a type of regulation of sarcomere organization [GO:0060297]; is a type of positive regulation of supramolecular fiber organization [GO:1902905]; positively regulates GO:0045214 Definition: Any process that increases the rate, frequency or extent of myofibril assembly by organization of muscle actomyosin into sarcomeres. The sarcomere is the repeating unit of a myofibril in a muscle cell, composed of an array of overlapping thick and thin filaments between two adjacent Z discs.